{
  "gene": "UniProtKB:Q8IVW8",
  "gene_symbol": "SPNS2",
  "gene_name": "Sphingosine-1-phosphate transporter SPNS2",
  "term_label": "sphingolipid transporter activity",
  "term_id": "GO:0046624"
}